{
  "term_id": "GO:0032922",
  "gene_symbol": "PASD1",
  "gene_name": "Circadian clock protein PASD1",
  "gene": "UniProtKB:Q8IV76",
  "term_label": "circadian regulation of gene expression"
}